{
  "gene_symbol": "PTPRO",
  "gene_name": "Receptor-type tyrosine-protein phosphatase O",
  "term_id": "GO:0005886",
  "gene": "UniProtKB:Q16827",
  "term_label": "plasma membrane"
}